{
  "gene_name": "LIM domain-containing protein 1",
  "term_label": "response to hypoxia",
  "term_id": "GO:0001666",
  "gene": "UniProtKB:Q9UGP4",
  "gene_symbol": "LIMD1"
}